{
  "term_id": "GO:1902018",
  "gene_symbol": "ODF2L",
  "gene_name": "Protein BCAP",
  "term_label": "negative regulation of cilium assembly",
  "gene": "UniProtKB:Q9ULJ1"
}